{
  "gene": "UniProtKB:P06310",
  "term_id": "UNKNOWN:0001",
  "term_label": "Unknown molecular function",
  "gene_symbol": "IGKV2-30",
  "gene_name": "Immunoglobulin kappa variable 2-30"
}